{
  "term_label": "lamellipodium",
  "gene_name": "Coronin-1A",
  "gene": "UniProtKB:P31146",
  "gene_symbol": "CORO1A",
  "term_id": "GO:0030027"
}